{
  "gene_symbol": "TMED10",
  "gene_name": "Transmembrane emp24 domain-containing protein 10",
  "term_id": "GO:0006888",
  "gene": "UniProtKB:P49755",
  "term_label": "endoplasmic reticulum to Golgi vesicle-mediated transport"
}